{
  "term_id": "GO:0035024",
  "gene_symbol": "KCTD10",
  "gene": "UniProtKB:Q9H3F6",
  "term_label": "negative regulation of Rho protein signal transduction",
  "gene_name": "BTB_POZ domain-containing adapter for CUL3-mediated RhoA degradation protein 3"
}